isoleucine transport [GO:0015818] (biological process) Sources: GOC:ai Also known as: L-isoleucine transport Subtypes: isoleucine transmembrane transport [GO:1903714] Definition: The directed movement of isoleucine, (2R*,3R*)-2-amino-3-methylpentanoic acid, into, out of or within a cell, or between cells, by means of some agent such as a transporter or pore. Relationships: is_a branched-chain amino acid transport [GO:0015803]; is a type of neutral amino acid transport [GO:0015804]